{
  "gene_symbol": "CHRNE",
  "gene_name": "Acetylcholine receptor subunit epsilon",
  "gene": "UniProtKB:Q04844",
  "term_label": "skeletal muscle contraction",
  "term_id": "GO:0003009"
}